{
  "term_id": "GO:0016020",
  "term_label": "membrane",
  "gene_name": "Olfactory receptor 2A7",
  "gene": "UniProtKB:Q96R45",
  "gene_symbol": "OR2A7"
}